{
  "gene_name": "Ankyrin repeat domain-containing protein 18A",
  "gene_symbol": "ANKRD18A",
  "term_id": "UNKNOWN:0003",
  "gene": "UniProtKB:Q8IVF6",
  "term_label": "Unknown cellular component"
}